{
  "term_label": "nucleus",
  "gene_name": "E3 ubiquitin-protein ligase RNF169",
  "term_id": "GO:0005634",
  "gene": "UniProtKB:Q8NCN4",
  "gene_symbol": "RNF169"
}